response to angiotensin [GO:1990776] (biological process) Definition: Any process that results in a change in state or activity of a cell or an organism (in terms of movement, secretion, enzyme production, gene expression, etc.) as a result of an angiotensin stimulus. Angiotensin is any of three physiologically active peptides (angiotensin II, III, or IV) processed from angiotensinogen. References: PMID:22982863 Subtypes: cellular response to angiotensin [GO:1904385] Relationships: is a type of response to peptide hormone [GO:0043434]